venom-mediated suppression of blood coagulation, intrinsic pathway [GO:0140184] (biological process) Definition: A process in which an organism inhibits or disrupts blood coagulation in another organism by suppression of the intrinsic pathway via the action of a venom. A common mechanism is the blocking the activity of host coagulation Factor XIIa (F12). References: PMID:25724270 Also known as: venom-mediated suppression of blood coagulation cascade, contact activation system Relationships: is a type of venom-mediated perturbation of biological process [GO:0035738]